{
  "gene_name": "Beta-citrylglutamate synthase B",
  "term_id": "UNKNOWN:0002",
  "term_label": "Unknown biological process",
  "gene_symbol": "RIMKLB",
  "gene": "UniProtKB:Q9ULI2"
}